{
  "term_label": "glycogenin glucosyltransferase activity",
  "term_id": "GO:0008466",
  "gene_symbol": "GYG1",
  "gene": "UniProtKB:P46976",
  "gene_name": "Glycogenin-1"
}